{
  "gene_symbol": "TYSND1",
  "term_label": "protein processing",
  "term_id": "GO:0016485",
  "gene": "UniProtKB:Q2T9J0",
  "gene_name": "Peroxisomal leader peptide-processing protease"
}